{
  "term_id": "GO:0042773",
  "gene": "UniProtKB:P00403",
  "gene_name": "Cytochrome c oxidase subunit 2",
  "term_label": "ATP synthesis coupled electron transport",
  "gene_symbol": "MT-CO2"
}